3alpha(S)-strictosidine biosynthetic process [GO:1901015] (biological process) Definition: The chemical reactions and pathways resulting in the formation of 3alpha(S)-strictosidine. Sources: GOC:TermGenie, GOC:yaf Also known as: 3alpha(S)-strictosidine metabolic process, 3alpha(S)-strictosidine anabolism, 3alpha(S)-strictosidine biosynthesis, 3alpha(S)-strictosidine formation, 3alpha(S)-strictosidine metabolism, 3alpha(S)-strictosidine synthesis Relationships: is a type of indole alkaloid biosynthetic process [GO:0035835]; is a type of beta-glucoside biosynthetic process [GO:1901806]